{
  "term_id": "GO:0005737",
  "gene_name": "NudC domain-containing protein 3",
  "gene_symbol": "NUDCD3",
  "gene": "UniProtKB:Q8IVD9",
  "term_label": "cytoplasm"
}